{
  "gene_symbol": "PABPC1L2A",
  "gene_name": "Polyadenylate-binding protein 1-like 2",
  "term_label": "poly(U) RNA binding",
  "term_id": "GO:0008266",
  "gene": "UniProtKB:Q5JQF8"
}